{
  "term_id": "GO:0005886",
  "gene": "UniProtKB:Q9Y5E3",
  "gene_symbol": "PCDHB6",
  "gene_name": "Protocadherin beta-6",
  "term_label": "plasma membrane"
}